basophil activation involved in immune response [GO:0002276] (biological process) Sources: GOC:add, ISBN:0781735149 Also known as: basophil activation during immune response Relationships: is a type of GO:0002366; is_a basophil activation [GO:0045575]; is part of myeloid cell activation involved in immune response [GO:0002275] Definition: A change in morphology and behavior of a basophil resulting from exposure to a cytokine, chemokine, soluble factor, or to (at least in mammals) an antigen which the basophil has specifically bound via IgE bound to Fc-epsilonRI receptors, leading to the initiation or perpetuation of an immune response.